{
  "gene_name": "Serine_threonine-protein kinase N2",
  "term_id": "UNKNOWN:0003",
  "gene": "UniProtKB:Q16513",
  "term_label": "Unknown cellular component",
  "gene_symbol": "PKN2"
}